{
  "term_label": "heparan sulfate proteoglycan catabolic process",
  "gene": "UniProtKB:P15586",
  "gene_name": "N-acetylglucosamine-6-sulfatase",
  "term_id": "GO:0030200",
  "gene_symbol": "GNS"
}